{
  "term_label": "Unknown molecular function",
  "term_id": "UNKNOWN:0001",
  "gene": "UniProtKB:Q6ZRM9",
  "gene_name": "Putative uncharacterized protein FLJ46235",
  "gene_symbol": "Q6ZRM9"
}